{
  "gene": "UniProtKB:A0A075B6W8",
  "term_id": "UNKNOWN:0003",
  "gene_name": "T cell receptor alpha joining 17 (Fragment)",
  "term_label": "Unknown cellular component",
  "gene_symbol": "TRAJ17"
}